{
  "term_id": "GO:0061640",
  "gene_name": "Dynactin subunit 3",
  "term_label": "cytoskeleton-dependent cytokinesis",
  "gene": "UniProtKB:O75935",
  "gene_symbol": "DCTN3"
}